{
  "term_label": "Unknown cellular component",
  "gene": "UniProtKB:Q96EZ4",
  "gene_symbol": "MYEOV",
  "gene_name": "Myeloma-overexpressed gene protein",
  "term_id": "UNKNOWN:0003"
}